skeletal muscle fiber development [GO:0048741] (biological process) Regulation: regulated by regulation of skeletal muscle fiber development [GO:0048742]; positively regulated by positive regulation of skeletal muscle fiber development [GO:0048743]; negatively regulated by negative regulation of skeletal muscle fiber development [GO:0048744] Relationships: is a type of myotube cell development [GO:0014904]; is part of skeletal muscle tissue development [GO:0007519] Sources: GOC:dph, GOC:ef, GOC:jid, GOC:lm, GOC:mtg_muscle Definition: The process whose specific outcome is the progression of the skeletal muscle fiber over time, from its formation to the mature structure. Muscle fibers are formed by the maturation of myotubes. They can be classed as slow, intermediate/fast or fast. Also known as: skeletal muscle fibre development, skeletal myofiber development, skeletal myofibre development